argininosuccinate lyase activity [GO:0004056] (molecular function) Definition: Catalysis of the reaction: N-(L-arginino)succinate = fumarate + L-arginine. Relationships: is a type of amidine-lyase activity [GO:0016842] Also known as: 2-(Nomega-L-arginino)succinate arginine-lyase (fumarate-forming), 2-(omega-N-L-arginino)succinate arginine-lyase (fumarate-forming), N-(L-argininosuccinate) arginine-lyase activity, arginine-succinate lyase activity, argininosuccinic acid lyase activity, arginosuccinase activity, omega-N-(L-arginino)succinate arginine-lyase activity Sources: EC:4.3.2.1